{
  "gene": "UniProtKB:O14638",
  "gene_name": "Ectonucleotide pyrophosphatase_phosphodiesterase family member 3",
  "term_label": "nucleoside triphosphate catabolic process",
  "gene_symbol": "ENPP3",
  "term_id": "GO:0009143"
}